{
  "gene_symbol": "SEC63",
  "gene": "UniProtKB:Q9UGP8",
  "term_label": "post-translational protein targeting to endoplasmic reticulum membrane",
  "gene_name": "Translocation protein SEC63 homolog",
  "term_id": "GO:0006620"
}